{
  "gene_name": "Zinc finger protein 25",
  "term_id": "GO:0006357",
  "term_label": "regulation of transcription by RNA polymerase II",
  "gene": "UniProtKB:P17030",
  "gene_symbol": "ZNF25"
}